{
  "gene_name": "Serine_threonine-protein phosphatase 2A 55 kDa regulatory subunit B beta isoform",
  "term_id": "GO:0019888",
  "gene": "UniProtKB:Q00005",
  "term_label": "protein phosphatase regulator activity",
  "gene_symbol": "PPP2R2B"
}